chemokine (C-C motif) ligand 22 production [GO:0071924] (biological process) Relationships: is a type of GO:0032602 References: PMID:18832724 Sources: GOC:mah Also known as: C-C motif chemokine 22 production, CCL-22 production, CCL22 production Definition: The appearance of chemokine (C-C motif) ligand 22 (CCL22) due to biosynthesis or secretion following a cellular stimulus, resulting in an increase in its intracellular or extracellular levels.